{
  "gene_symbol": "PITX2",
  "gene_name": "Pituitary homeobox 2",
  "term_label": "RNA polymerase II cis-regulatory region sequence-specific DNA binding",
  "term_id": "GO:0000978",
  "gene": "UniProtKB:Q99697"
}